{
  "term_id": "UNKNOWN:0002",
  "term_label": "Unknown biological process",
  "gene": "UniProtKB:O14548",
  "gene_name": "Cytochrome c oxidase subunit 7A-related protein, mitochondrial",
  "gene_symbol": "COX7A2L"
}